{
  "gene": "UniProtKB:Q9H0A0",
  "term_label": "tRNA binding",
  "term_id": "GO:0000049",
  "gene_symbol": "NAT10",
  "gene_name": "RNA cytidine acetyltransferase"
}